axonemal dynein complex [GO:0005858] (cellular component) Subtypes: inner dynein arm [GO:0036156], outer dynein arm [GO:0036157] Definition: A dynein complex found in eukaryotic cilia and flagella; the motor domain heads interact with adjacent microtubules to generate a sliding force which is converted to a bending motion. Sources: GOC:cilia, GOC:hla, GOC:krc, ISBN:0815316194 Also known as: axonemal dynein heavy chain, axonemal dynein intermediate chain, axonemal dynein intermediate light chain, axonemal dynein light chain Relationships: is a type of dynein complex [GO:0030286]; is part of axoneme [GO:0005930]